{
  "gene_name": "Sorting nexin-4",
  "term_label": "protein transport",
  "gene_symbol": "SNX4",
  "gene": "UniProtKB:O95219",
  "term_id": "GO:0015031"
}